{
  "gene_symbol": "OSBP2",
  "term_label": "plasma membrane",
  "term_id": "GO:0005886",
  "gene": "UniProtKB:Q969R2",
  "gene_name": "Oxysterol-binding protein 2"
}